{
  "gene_name": "Electrogenic aspartate_glutamate antiporter SLC25A13, mitochondrial",
  "term_id": "GO:0015813",
  "gene": "UniProtKB:Q9UJS0",
  "term_label": "L-glutamate transmembrane transport",
  "gene_symbol": "SLC25A13"
}